{
  "gene_name": "Elongator complex protein 4",
  "term_id": "GO:0002098",
  "gene": "UniProtKB:Q96EB1",
  "term_label": "tRNA wobble uridine modification",
  "gene_symbol": "ELP4"
}